positive regulation of androgen secretion [GO:2000836] (biological process) Definition: Any process that activates or increases the frequency, rate or extent of androgen secretion. Sources: GOC:sl Relationships: is_a positive regulation of steroid hormone secretion [GO:2000833]; is a type of GO:2000834; positively regulates androgen secretion [GO:0035935]